negative regulation of pancreatic A cell differentiation [GO:2000227] (biological process) Relationships: is a type of negative regulation of epithelial cell differentiation [GO:0030857]; is a type of GO:0051241; is a type of regulation of pancreatic A cell differentiation [GO:2000226]; negatively regulates pancreatic A cell differentiation [GO:0003310] Also known as: negative regulation of pancreatic alpha cell differentiation Sources: GOC:mah Definition: Any process that stops, prevents, or reduces the frequency, rate or extent of pancreatic A cell differentiation.